negative regulation of neuron apoptotic process [GO:0043524] (biological process) Subtypes: negative regulation of hippocampal neuron apoptotic process [GO:0110091], negative regulation of oxidative stress-induced neuron intrinsic apoptotic signaling pathway [GO:1903377], GO:1903382, negative regulation of outer hair cell apoptotic process [GO:1905586], GO:2000672 Definition: Any process that stops, prevents, or reduces the frequency, rate or extent of cell death by apoptotic process in neurons. Sources: GOC:go_curators, GOC:mtg_apoptosis Also known as: down regulation of neuron apoptosis, down-regulation of neuron apoptosis, downregulation of neuron apoptosis, negative regulation of programmed cell death, neurons, inhibition of neuron apoptosis, negative regulation of neuron apoptosis, neuron survival Relationships: is_a GO:0043066; is_a regulation of neuron apoptotic process [GO:0043523]; negatively regulates neuron apoptotic process [GO:0051402]